{
  "gene_name": "NADH-ubiquinone oxidoreductase chain 6",
  "term_id": "UNKNOWN:0002",
  "gene": "UniProtKB:P03923",
  "term_label": "Unknown biological process",
  "gene_symbol": "MT-ND6"
}